baicalein 7-O-glucuronosyltransferase activity [GO:0102159] (molecular function) Definition: Catalysis of the reaction: UDP-alpha-D-glucuronate + baicalein = H+ + UDP + baicalin. Sources: RHEA:28314 Relationships: is a type of hexosyltransferase activity [GO:0016758]